{
  "term_id": "UNKNOWN:0002",
  "gene": "UniProtKB:O15018",
  "term_label": "Unknown biological process",
  "gene_symbol": "PDZD2",
  "gene_name": "PDZ domain-containing protein 2"
}